{
  "gene_name": "AP-5 complex subunit zeta-1",
  "term_label": "Unknown molecular function",
  "term_id": "UNKNOWN:0001",
  "gene": "UniProtKB:O43299",
  "gene_symbol": "AP5Z1"
}